{
  "gene_symbol": "OPA3",
  "term_label": "mitochondrion",
  "term_id": "GO:0005739",
  "gene": "UniProtKB:Q9H6K4",
  "gene_name": "Optic atrophy 3 protein"
}